{
  "gene_name": "Zinc finger CCCH domain-containing protein 14",
  "gene": "UniProtKB:Q6PJT7",
  "gene_symbol": "ZC3H14",
  "term_label": "regulation of mRNA stability",
  "term_id": "GO:0043488"
}